{
  "gene_symbol": "PHOX2B",
  "gene": "UniProtKB:Q99453",
  "term_id": "GO:0005634",
  "term_label": "nucleus",
  "gene_name": "Paired mesoderm homeobox protein 2B"
}